{
  "term_id": "GO:0005739",
  "gene_symbol": "ISCA1",
  "gene_name": "Iron-sulfur cluster assembly 1 homolog, mitochondrial",
  "term_label": "mitochondrion",
  "gene": "UniProtKB:Q9BUE6"
}